{
  "gene": "UniProtKB:Q96IF1",
  "term_id": "GO:0035331",
  "gene_name": "LIM domain-containing protein ajuba",
  "term_label": "negative regulation of hippo signaling",
  "gene_symbol": "AJUBA"
}